{
  "gene_symbol": "PBLD",
  "term_id": "UNKNOWN:0001",
  "term_label": "Unknown molecular function",
  "gene_name": "Phenazine biosynthesis-like domain-containing protein",
  "gene": "UniProtKB:P30039"
}